{
  "term_id": "GO:0051015",
  "gene_symbol": "MYH6",
  "gene_name": "Myosin-6",
  "gene": "UniProtKB:P13533",
  "term_label": "actin filament binding"
}